{
  "gene_symbol": "PABPC4L",
  "gene_name": "Polyadenylate-binding protein 4-like",
  "gene": "UniProtKB:P0CB38",
  "term_label": "ribonucleoprotein complex",
  "term_id": "GO:1990904"
}